{
  "term_label": "spermatid development",
  "term_id": "GO:0007286",
  "gene_symbol": "ZMYND15",
  "gene": "UniProtKB:Q9H091",
  "gene_name": "Zinc finger MYND domain-containing protein 15"
}